{
  "term_id": "GO:0051919",
  "term_label": "positive regulation of fibrinolysis",
  "gene_name": "Plasma kallikrein",
  "gene": "UniProtKB:P03952",
  "gene_symbol": "KLKB1"
}